{
  "gene": "UniProtKB:Q92886",
  "gene_name": "Neurogenin-1",
  "gene_symbol": "NEUROG1",
  "term_label": "DNA-binding transcription factor activity, RNA polymerase II-specific",
  "term_id": "GO:0000981"
}